chemoattraction involved in precerebellar neuron migration [GO:0021951] (biological process) Definition: The creation and reception of signals that guide a precerebellar neuron towards their signals, where this process is involved in tangential migration. Also known as: positive chemotaxis involved in precerebellar neuron migration Relationships: is a type of positive chemotaxis [GO:0050918]; is part of brainstem precerebellar neuron precursor migration [GO:0021949] References: PMID:15157725 Sources: GOC:cls, GOC:dgh, GOC:dph, GOC:jid, GO_REF:0000021